lateral element [GO:0000800] (CC) Also known as: axial element Relationships: is a type of cellular anatomical structure [GO:0110165]; is part of synaptonemal complex [GO:0000795] Note: In species that have a synaptonemal complex, the lateral elements are part of this complex. S.pombe is an example of a species that lacks a (canonical) synaptonemal complex, but still has lateral elements. Definition: A proteinaceous core found between sister chromatids during meiotic prophase. Sources: GOC:elh